{
  "gene": "UniProtKB:Q86SY8",
  "term_label": "Unknown biological process",
  "gene_name": "Putative uncharacterized protein KTN1-AS1",
  "gene_symbol": "KTN1-AS1",
  "term_id": "UNKNOWN:0002"
}